doxorubicin transport [GO:1900753] (BP) Also known as: (1S,3S)-3,5,12-trihydroxy-3-(hydroxyacetyl)-10-methoxy-6,11-dioxo-1,2,3,4,6,11-hexahydrotetracen-1-yl 3-amino-2,3,6-trideoxy-alpha-L-lyxo-hexopyranoside transport, (1S,3S)-3-glycoloyl-3,5,12-trihydroxy-10-methoxy-6,11-dioxo-1,2,3,4,6,11-hexahydrotetracen-1-yl 3-amino-2,3,6-trideoxy-alpha-L-lyxo-hexopyranoside transport, (8S-cis)-10-((3-amino-2,3,6-trideoxy-alpha-L-lyxo-hexopyranosyl)oxy)-7,8,9,10-tetrahydro-6,8,11-trihydroxy-8-(hydroxyacetyl)-1-methoxy-5,12-naphthacenedione transport, 14-hydroxydaunomycin transport, 14-hydroxydaunorubicine transport, Adriamycin transport, doxorubicine transport, doxorubicinum transport References: PMID:12057006, PMID:15090538, PMID:19063901, PMID:19651502, PMID:9651400 Sources: GOC:TermGenie Definition: The directed movement of a doxorubicin into, out of or within a cell, or between cells, by means of some agent such as a transporter or pore. Relationships: is_a organic cation transport [GO:0015695]; is a type of GO:0015850; is a type of nitrogen compound transport [GO:0071705]; is a type of glycoside transport [GO:1901656]